positive regulation of syringal lignin biosynthetic process [GO:1901430] (biological process) Sources: GOC:TermGenie Relationships: is a type of positive regulation of secondary metabolite biosynthetic process [GO:1900378]; is a type of GO:1901428; RO_0002213 syringal lignin biosynthetic process [GO:1901066] Also known as: activation of S-lignin biosynthetic process, activation of syringal lignin anabolism, activation of syringal lignin biosynthesis, activation of syringal lignin formation, activation of syringal lignin synthesis, positive regulation of S-lignin biosynthetic process, positive regulation of syringal lignin anabolism, positive regulation of syringal lignin biosynthesis, positive regulation of syringal lignin formation, positive regulation of syringal lignin synthesis, up regulation of S-lignin biosynthetic process, up regulation of syringal lignin anabolism, up regulation of syringal lignin biosynthesis, up regulation of syringal lignin biosynthetic process, up regulation of syringal lignin formation, up regulation of syringal lignin synthesis, up-regulation of S-lignin biosynthetic process, up-regulation of syringal lignin anabolism, up-regulation of syringal lignin biosynthesis, up-regulation of syringal lignin biosynthetic process, up-regulation of syringal lignin formation, up-regulation of syringal lignin synthesis, upregulation of S-lignin biosynthetic process, upregulation of syringal lignin anabolism, upregulation of syringal lignin biosynthesis, upregulation of syringal lignin biosynthetic process, upregulation of syringal lignin formation, upregulation of syringal lignin synthesis, activation of syringal lignin biosynthetic process Definition: Any process that activates or increases the frequency, rate or extent of syringal lignin biosynthetic process.